{
  "gene": "UniProtKB:Q7Z7J7",
  "term_id": "GO:0045211",
  "gene_name": "LHFPL tetraspan subfamily member 4 protein",
  "gene_symbol": "LHFPL4",
  "term_label": "postsynaptic membrane"
}